specification of nephron tubule identity [GO:0072081] (biological process) Relationships: is a type of GO:0007379; is a type of pattern specification involved in kidney development [GO:0061004]; is part of GO:0072047; is part of GO:0072079 Subtypes: GO:0039005, specification of mesonephric nephron tubule identity [GO:0061282], specification of proximal tubule identity [GO:0072082], specification of distal tubule identity [GO:0072084], specification of connecting tubule identity [GO:0072085], specification of loop of Henle identity [GO:0072086], specification of mesonephric tubule identity [GO:0072167], GO:0072293 Definition: The process in which the tubules arranged along the proximal/distal axis of the nephron acquire their identity. Sources: GOC:bf, GOC:mtg_kidney_jan10